long-chain fatty acid transport [GO:0015909] (biological process) Subtypes: carnitine shuttle [GO:0006853], long-chain fatty acid import into peroxisome [GO:0015910], long-chain fatty acid import into cell [GO:0044539], arachidonate transport [GO:1903963] Sources: GOC:ai Note: While there is not universal consensus on the lengths of short-, medium-, long- and very-long-chain fatty acids, the GO uses the definitions in ChEBI (see CHEBI:26666, CHEBI:59554, CHEBI:15904 and CHEBI:27283). Definition: The directed movement of a long-chain fatty acid into, out of or within a cell, or between cells, by means of some agent such as a transporter or pore. A long-chain fatty acid has an aliphatic tail containing 13 to 22 carbons. Relationships: is a type of fatty acid transport [GO:0015908]